FAD-AMP lyase (cyclizing) activity [GO:0034012] (molecular function) Also known as: FAD AMP-lyase (cyclic-FMN-forming) activity, FAD AMP-lyase (riboflavin-cyclic-4',5'-phosphate-forming) activity, FMN cyclase activity Sources: RHEA:13729 Definition: Catalysis of the reaction: FAD = AMP + H+ + riboflavin cyclic-4',5'-phosphate. Relationships: is a type of cyclase activity [GO:0009975]; is a type of phosphorus-oxygen lyase activity [GO:0016849]